establishment of protein localization to postsynaptic membrane [GO:1903540] (biological process) Definition: The directed movement of a protein to a specific location in a postsynaptic membrane. Relationships: is a type of establishment of protein localization to membrane [GO:0090150] Subtypes: neurotransmitter receptor transport to postsynaptic membrane [GO:0098969] Also known as: establishment of protein localisation in postsynaptic membrane, establishment of protein localisation to postsynaptic membrane, establishment of protein localization in postsynaptic membrane References: PMID:9753322 Sources: GOC:TermGenie, GOC:kmv, GO_REF:0000087